positive regulation of R7 cell fate commitment [GO:0106397] (biological process) Definition: Any process that activates or increases the frequency, rate or extent of R7 cell fate commitment. References: PMID:22878552 Sources: GOC:ha Relationships: is a type of positive regulation of cell fate commitment [GO:0010455]; is a type of regulation of R7 cell fate commitment [GO:0106396]; positively regulates R7 cell fate commitment [GO:0007465]